{
  "gene_symbol": "CENPF",
  "term_label": "dynein complex binding",
  "gene_name": "Centromere protein F",
  "gene": "UniProtKB:P49454",
  "term_id": "GO:0070840"
}